{
  "gene_name": "P antigen family member 5",
  "term_id": "UNKNOWN:0003",
  "gene": "UniProtKB:Q96GU1",
  "term_label": "Unknown cellular component",
  "gene_symbol": "PAGE5"
}